{
  "gene": "UniProtKB:P32239",
  "gene_symbol": "CCKBR",
  "term_id": "GO:0007218",
  "term_label": "neuropeptide signaling pathway",
  "gene_name": "Gastrin_cholecystokinin type B receptor"
}